{
  "gene_name": "Large ribosomal subunit protein uL1",
  "gene": "UniProtKB:P62906",
  "term_label": "Unknown biological process",
  "term_id": "UNKNOWN:0002",
  "gene_symbol": "RPL10A"
}